{
  "gene_name": "Doublesex- and mab-3-related transcription factor A1",
  "gene_symbol": "DMRTA1",
  "term_label": "RNA polymerase II cis-regulatory region sequence-specific DNA binding",
  "term_id": "GO:0000978",
  "gene": "UniProtKB:Q5VZB9"
}